{
  "gene": "UniProtKB:Q5T036",
  "term_id": "UNKNOWN:0003",
  "gene_symbol": "FAM120AOS",
  "gene_name": "Uncharacterized protein FAM120AOS",
  "term_label": "Unknown cellular component"
}